{
  "gene_name": "Lysine-specific demethylase 4A",
  "gene_symbol": "KDM4A",
  "term_id": "GO:0000785",
  "term_label": "chromatin",
  "gene": "UniProtKB:O75164"
}